guanine biosynthetic process [GO:0046099] (biological process) Relationships: is a type of purine nucleobase biosynthetic process [GO:0009113]; is a type of guanine metabolic process [GO:0046098] Also known as: guanine anabolism, guanine biosynthesis, guanine formation, guanine synthesis Sources: GOC:go_curators Subtypes: GO:0006178 Definition: The chemical reactions and pathways resulting in the formation of guanine, 2-amino-6-hydroxypurine, a purine that is one of the five main bases found in nucleic acids and a component of a number of phosphorylated guanosine derivatives whose metabolic or regulatory functions are important.